{
  "term_id": "GO:0016477",
  "gene": "UniProtKB:Q86YL7",
  "gene_name": "Podoplanin",
  "gene_symbol": "PDPN",
  "term_label": "cell migration"
}